1,2-dihydroxy-6-methylcyclohexa-3,5-dienecarboxylate dehydrogenase activity [GO:0018521] (molecular function) Also known as: 1,2-dihydroxy-6-methylcyclohexa-3,5-dienecarboxylate:NAD+ oxidoreductase (decarboxylating) Relationships: is a type of oxidoreductase activity, acting on the CH-CH group of donors, NAD or NADP as acceptor [GO:0016628] Definition: Catalysis of the reaction: 1,6-dihydroxy-2-methylcyclohexa-2,4-dienecarboxylate + NAD+ = 3-methylcatechol + CO2 + NADH. Sources: EC:1.3.1.68, RHEA:15657